{
  "gene": "UniProtKB:Q0VAQ4",
  "gene_symbol": "SMAGP",
  "gene_name": "Small cell adhesion glycoprotein",
  "term_id": "UNKNOWN:0002",
  "term_label": "Unknown biological process"
}